phosphatidylinositol 3-kinase complex, class III, type II [GO:0034272] (cellular component) Also known as: PtdIns-3-kinase complex II, phosphatidylinositol 3-kinase complex II References: PMID:11157979, PMID:16421251 Sources: GOC:ha, GOC:rb Note: Note that this term should not be confused with '1-phosphatidylinositol-4-phosphate 3-kinase, class IA complex; GO:0005943' or '1-phosphatidylinositol-4-phosphate 3-kinase, class IB complex ; GO:0005944'. Relationships: is a type of phosphatidylinositol 3-kinase complex, class III [GO:0035032] Definition: A class III phosphatidylinositol 3-kinase complex that is involved in vacuolar protein sorting (VPS) via endosomes. In budding yeast, this complex consists of Vps30p, Vps34p, Vps38 and Vps15p.